{
  "gene": "UniProtKB:P42765",
  "term_id": "GO:0003985",
  "gene_name": "3-ketoacyl-CoA thiolase, mitochondrial",
  "gene_symbol": "ACAA2",
  "term_label": "acetyl-CoA C-acetyltransferase activity"
}